fatty acyl-[ACP] hydrolase activity [GO:0016297] (molecular function) Definition: Catalysis of the reaction: a fatty acyl-[ACP] + H2O = a fatty acid + H+ + holo-[acyl-carrier protein]. Sources: RHEA:44596 Relationships: is a type of thiolester hydrolase activity [GO:0016790] Also known as: acyl-ACP hydrolase activity, acyl-ACP thioesterase activity, acyl-[acyl-carrier protein] hydrolase activity, acyl-[acyl-carrier-protein] hydrolase activity, acyl-ACP-hydrolase activity, acyl-acyl carrier protein hydrolase activity, acyl-acyl-carrier-protein hydrolase activity